protein localization to cell cortex [GO:0072697] (biological process) Regulation: regulated by regulation of protein localization to cell cortex [GO:1904776]; negatively regulated by negative regulation of protein localization to cell cortex [GO:1904777]; positively regulated by positive regulation of protein localization to cell cortex [GO:1904778] Subtypes: protein localization to actin cortical patch [GO:0044379], protein localization to medial cortex [GO:0071574], protein localization to cortical microtubule cytoskeleton [GO:0072699], GO:0097446, protein localization to septin ring [GO:1902935], protein localization to lateral cortical node [GO:1903360], protein localization to cortical endoplasmic reticulum [GO:1903419], GO:1990179, protein localization to cell cortex of cell tip [GO:1990896] Definition: A process in which a protein is transported to, or maintained in, the cell cortex. Also known as: protein localisation to cell cortex Relationships: is a type of protein localization to cell periphery [GO:1990778] Sources: GOC:mah